pancreatic epsilon cell differentiation [GO:0090104] (biological process) Definition: The process in which relatively unspecialized cells acquire specialized structural and functional features of a pancreatic epsilon cell. A pancreatic epsilon cell is a cell in the pancreas that secretes ghrelin. Sources: GOC:dph, GOC:tb Also known as: pancreatic E cell differentiation Relationships: is a type of enteroendocrine cell differentiation [GO:0035883]; is part of endocrine pancreas development [GO:0031018]